{
  "gene_name": "CCAAT_enhancer-binding protein beta",
  "term_id": "GO:0045595",
  "term_label": "regulation of cell differentiation",
  "gene": "UniProtKB:P17676",
  "gene_symbol": "CEBPB"
}